{
  "gene_name": "Trafficking kinesin-binding protein 2",
  "gene": "UniProtKB:O60296",
  "gene_symbol": "TRAK2",
  "term_label": "myosin binding",
  "term_id": "GO:0017022"
}